negative adaptation of signaling pathway by response to pheromone involved in pheromone-induced unidirectional conjugation [GO:0000766] (biological process) Sources: GOC:clt Definition: In organisms that undergo pheromone-induced unidirectional conjugation, the process involved in desensitization following exposure to pheromone stimulus that acts to down-regulate further stimulation or block initial conjugation responses. Relationships: is a type of negative adaptation of signaling pathway [GO:0022401]; is part of response to pheromone regulating pheromone-induced unidirectional conjugation [GO:0000765] Also known as: desensitization to pheromone during pheromone-induced unidirectional conjugation, negative adaptation of signalling pathway by response to pheromone involved in pheromone-induced unidirectional conjugation, adaptation to pheromone during pheromone-induced unidirectional conjugation